{
  "gene": "UniProtKB:P16444",
  "term_id": "UNKNOWN:0002",
  "gene_name": "Dipeptidase 1",
  "gene_symbol": "DPEP1",
  "term_label": "Unknown biological process"
}